macrophomate synthase activity [GO:0033191] (molecular function) Definition: Catalysis of the reaction: a 2-pyrone + oxalacetate = macrophomate. References: PMID:10984474 Sources: GOC:cb Relationships: is a type of GO:0016744